{
  "gene": "UniProtKB:Q5T4I8",
  "term_label": "Unknown molecular function",
  "gene_name": "Putative uncharacterized protein C6orf52",
  "gene_symbol": "C6orf52",
  "term_id": "UNKNOWN:0001"
}